regulation of imaginal disc-derived wing vein specification [GO:0110107] (BP) References: PMID:11861482 Sources: GOC:ha Relationships: is a type of GO:0051239; regulates imaginal disc-derived wing vein specification [GO:0007474] Definition: Any process that modulates the frequency, rate or extent of imaginal disc-derived wing vein specification. Subtypes: positive regulation of imaginal disc-derived wing vein specification [GO:0110108], negative regulation of imaginal disc-derived wing vein specification [GO:0110109]